{
  "gene_symbol": "PLPP3",
  "term_label": "sphingosine-1-phosphate phosphatase activity",
  "gene": "UniProtKB:O14495",
  "term_id": "GO:0042392",
  "gene_name": "Phospholipid phosphatase 3"
}